{
  "gene_symbol": "CTNNA1",
  "gene_name": "Catenin alpha-1",
  "gene": "UniProtKB:P35221",
  "term_id": "GO:0005912",
  "term_label": "adherens junction"
}